{
  "gene_symbol": "DPP10",
  "term_label": "plasma membrane",
  "gene_name": "Inactive dipeptidyl peptidase 10",
  "term_id": "GO:0005886",
  "gene": "UniProtKB:Q8N608"
}